{
  "gene_symbol": "DPH1",
  "gene": "UniProtKB:Q9BZG8",
  "gene_name": "2-(3-amino-3-carboxypropyl)histidine synthase subunit 1",
  "term_label": "Unknown molecular function",
  "term_id": "UNKNOWN:0001"
}